24-methylenesterol C-methyltransferase activity [GO:0030797] (molecular function) Definition: Catalysis of the reaction: 24-methylidenelophenol + S-adenosyl-L-methionine(1+) = (Z)-24-ethylidenelophenol + S-adenosyl-L-homocysteine + H+. Sources: EC:2.1.1.143, RHEA:21044 Also known as: SMT(2) activity, 24-methylenelophenol C-24(1)-methyltransferase activity, 24-methylenelophenol C-241-methyltransferase activity, S-adenosyl-L-methionine:24-methylenelophenol C-methyltransferase activity, SMT2 Relationships: is a type of GO:0008757